{
  "term_id": "GO:0036041",
  "gene_name": "Fatty acid-binding protein 9",
  "term_label": "long-chain fatty acid binding",
  "gene": "UniProtKB:Q0Z7S8",
  "gene_symbol": "FABP9"
}